pyranose oxidase activity [GO:0050233] (molecular function) Sources: EC:1.1.3.10, RHEA:10552 Relationships: is a type of oxidoreductase activity, acting on the CH-OH group of donors, oxygen as acceptor [GO:0016899] Also known as: glucose 2-oxidase activity, pyranose-2-oxidase activity, pyranose:oxygen 2-oxidoreductase activity Definition: Catalysis of the reaction: D-glucose + O2 = 2-dehydro-D-glucose + H2O2.